{
  "term_label": "embryonic skeletal system morphogenesis",
  "gene_name": "Homeobox protein Hox-B4",
  "term_id": "GO:0048704",
  "gene_symbol": "HOXB4",
  "gene": "UniProtKB:P17483"
}